{
  "term_id": "GO:0000445",
  "term_label": "THO complex part of transcription export complex",
  "gene_symbol": "THOC1",
  "gene_name": "THO complex subunit 1",
  "gene": "UniProtKB:Q96FV9"
}